urokinase plasminogen activator receptor activity [GO:0030377] (molecular function) Definition: Combining with the urokinase plasminogen activator to initiate a change in cell activity. References: PMID:16456079 Sources: GOC:mah Relationships: is a type of signaling receptor activity [GO:0038023]; is part of urokinase plasminogen activator signaling pathway [GO:0038195] Also known as: U-plasminogen activator receptor activity, uPAR, urokinase plasminogen activator receptor